{
  "term_id": "GO:0051014",
  "gene": "UniProtKB:P06396",
  "gene_name": "Gelsolin",
  "term_label": "actin filament severing",
  "gene_symbol": "GSN"
}